{
  "gene_name": "THAP domain-containing protein 3",
  "gene": "UniProtKB:Q8WTV1",
  "term_label": "Unknown molecular function",
  "term_id": "UNKNOWN:0001",
  "gene_symbol": "THAP3"
}